{
  "term_label": "phospholipase C-activating G protein-coupled receptor signaling pathway",
  "gene_name": "Alpha-1B adrenergic receptor",
  "term_id": "GO:0007200",
  "gene_symbol": "ADRA1B",
  "gene": "UniProtKB:P35368"
}